D-allose kinase activity [GO:0008787] (molecular function) Definition: Catalysis of the reaction: ATP + D-allose = ADP + D-allose 6-phosphate. Also known as: allose kinase activity, ATP:D-allose 6-phosphotransferase activity, D-allokinase activity, D-allose-6-kinase activity, allokinase (phosphorylating), allokinase activity Sources: EC:2.7.1.55 Relationships: is a type of hexokinase activity [GO:0004396]